{
  "gene_symbol": "MUC17",
  "term_label": "apical plasma membrane",
  "gene_name": "Mucin-17",
  "gene": "UniProtKB:Q685J3",
  "term_id": "GO:0016324"
}